{
  "term_label": "external side of plasma membrane",
  "gene_symbol": "BTNL10P",
  "gene_name": "Putative butyrophilin-like protein 10 pseudogene",
  "gene": "UniProtKB:A8MVZ5",
  "term_id": "GO:0009897"
}